{
  "term_id": "UNKNOWN:0002",
  "gene": "UniProtKB:P0C626",
  "gene_name": "Olfactory receptor 5G3",
  "gene_symbol": "OR5G3",
  "term_label": "Unknown biological process"
}